angiotensin-mediated drinking behavior [GO:0003051] (biological process) Sources: GOC:mtg_cardio Relationships: is a type of drinking behavior [GO:0042756]; BFO_0000050 brain renin-angiotensin system [GO:0002035] Also known as: angiotensin mediated drinking behavior Definition: The drinking behavior that is mediated by the action of angiotensin in the brain. Angiotensin stimulates the brain centers that control thirst.